{
  "term_id": "GO:0016020",
  "gene_symbol": "TMEM131",
  "gene_name": "Transmembrane protein 131",
  "term_label": "membrane",
  "gene": "UniProtKB:Q92545"
}